egg coat [GO:0035805] (cellular component) Relationships: is a type of GO:0140047 References: PMID:16944418, PMID:17163408 Also known as: vitelline membrane, zona pellucida Subtypes: fertilization envelope [GO:0060387], vitelline envelope [GO:0060388] Definition: A specialized extracellular matrix that surrounds the plasma membrane of the ovum of animals. The egg coat provides structural support and can play an essential role in oogenesis, fertilization and early development.